{
  "gene_symbol": "STAC2",
  "gene": "UniProtKB:Q6ZMT1",
  "term_label": "Unknown molecular function",
  "term_id": "UNKNOWN:0001",
  "gene_name": "SH3 and cysteine-rich domain-containing protein 2"
}